{
  "gene_name": "Olfactory receptor 56B4",
  "gene_symbol": "OR56B4",
  "term_label": "plasma membrane",
  "term_id": "GO:0005886",
  "gene": "UniProtKB:Q8NH76"
}